{
  "term_id": "UNKNOWN:0001",
  "gene_symbol": "MSMB",
  "gene_name": "Beta-microseminoprotein",
  "gene": "UniProtKB:P08118",
  "term_label": "Unknown molecular function"
}